{
  "gene_symbol": "DHX9",
  "gene": "UniProtKB:Q08211",
  "term_label": "3'-5' DNA helicase activity",
  "gene_name": "ATP-dependent RNA helicase A",
  "term_id": "GO:0043138"
}